{
  "term_id": "UNKNOWN:0003",
  "gene": "UniProtKB:Q92185",
  "gene_symbol": "ST8SIA1",
  "gene_name": "Alpha-N-acetylneuraminide alpha-2,8-sialyltransferase",
  "term_label": "Unknown cellular component"
}